negative regulation of response to amylopectin [GO:1900522] (biological process) Definition: Any process that stops, prevents or reduces the frequency, rate or extent of response to amylopectin. Sources: GOC:TermGenie, GOC:mengo_curators Also known as: down regulation of response to amylopectin, down-regulation of response to amylopectin, downregulation of response to amylopectin, inhibition of response to amylopectin Relationships: is a type of negative regulation of response to stimulus [GO:0048585]; is_a regulation of response to amylopectin [GO:1900521]; negatively regulates response to amylopectin [GO:0044591]